EGFR:ERBB2 complex [GO:0038142] (cellular component) Relationships: is a type of plasma membrane signaling receptor complex [GO:0098802] References: PMID:16460914, PMID:1973074 Sources: GOC:signaling Definition: A heterodimeric complex between the tyrosine kinase receptor ERBB2 and a ligand-activated epidermal growth factor receptor (EGFR/ERBB1). ERBB2, which does not bind any known ligand, is activated through formation of a heterodimer with another ligand-activated ERBB family member such as EGFR. Also known as: EGF:EGFR:ERBB2 complex, EGFR:ERBB2 heterodimer